negative regulation of steroid hormone secretion [GO:2000832] (biological process) Subtypes: negative regulation of ecdysteroid secretion [GO:0045999], negative regulation of androgen secretion [GO:2000835], negative regulation of corticosteroid hormone secretion [GO:2000847], negative regulation of estrogen secretion [GO:2000862], negative regulation of estradiol secretion [GO:2000865], GO:2000868, negative regulation of progesterone secretion [GO:2000871] Definition: Any process that stops, prevents or reduces the frequency, rate or extent of steroid hormone secretion. Sources: GOC:sl Relationships: is a type of negative regulation of lipid transport [GO:0032369]; is_a GO:0046888; is a type of negative regulation of multicellular organismal process [GO:0051241]; is a type of regulation of steroid hormone secretion [GO:2000831]; RO_0002212 steroid hormone secretion [GO:0035929]